{
  "gene_symbol": "AURKA",
  "term_id": "GO:0005813",
  "term_label": "centrosome",
  "gene_name": "Aurora kinase A",
  "gene": "UniProtKB:O14965"
}